{
  "gene_name": "ATP-dependent DNA helicase Q4",
  "gene_symbol": "RECQL4",
  "term_label": "nucleus",
  "term_id": "GO:0005634",
  "gene": "UniProtKB:O94761"
}